{
  "term_id": "GO:0016010",
  "gene_name": "Beta-2-syntrophin",
  "term_label": "dystrophin-associated glycoprotein complex",
  "gene_symbol": "SNTB2",
  "gene": "UniProtKB:Q13425"
}